paxilline biosynthetic process [GO:0140873] (biological process) Also known as: paxilline anabolism, paxilline biosynthesis, paxilline formation, paxilline synthesis Definition: The chemical reactions and pathways resulting in the formation of paxilline, a mycotoxin that acts as an inhibitor of mammalian maxi-K channels. Relationships: is a type of terpenoid indole alkaloid biosynthetic process [GO:0009709]; is a type of diterpenoid biosynthetic process [GO:0016102]; is a type of GO:0042181; is a type of GO:0043386; is a type of GO:0120255; is a type of tertiary alcohol biosynthetic process [GO:1902645] References: PMID:23949005